{
  "term_label": "Unknown biological process",
  "gene_name": "Alpha-tectorin",
  "term_id": "UNKNOWN:0002",
  "gene": "UniProtKB:O75443",
  "gene_symbol": "TECTA"
}